{
  "gene_name": "Myotubularin-related protein 1",
  "term_label": "membrane",
  "term_id": "GO:0016020",
  "gene": "UniProtKB:Q13613",
  "gene_symbol": "MTMR1"
}